{
  "gene": "UniProtKB:Q9Y6X4",
  "gene_symbol": "FAM169A",
  "term_label": "Unknown cellular component",
  "term_id": "UNKNOWN:0003",
  "gene_name": "Soluble lamin-associated protein of 75 kDa"
}